{
  "gene_name": "Phosphoinositide 3-kinase regulatory subunit 4",
  "gene": "UniProtKB:Q99570",
  "term_id": "GO:0005770",
  "gene_symbol": "PIK3R4",
  "term_label": "late endosome"
}